3-hydroxybenzoate 4-monooxygenase activity [GO:0018668] (molecular function) Sources: EC:1.14.13.23, RHEA:11480 Also known as: 3-hydroxybenzoate 4-hydroxylase activity, 3-hydroxybenzoate,NADPH:oxygen oxidoreductase (4-hydroxylating) Definition: Catalysis of the reaction: 3-hydroxybenzoate + H+ + NADPH + O2 = 3,4-dihydroxybenzoate + H2O + NADP+. Relationships: is a type of oxidoreductase activity, acting on paired donors, with incorporation or reduction of molecular oxygen, NAD(P)H as one donor, and incorporation of one atom of oxygen [GO:0016709]